{
  "term_label": "DNA-binding transcription factor activity, RNA polymerase II-specific",
  "gene_name": "Homeobox protein cut-like 2",
  "gene": "UniProtKB:O14529",
  "term_id": "GO:0000981",
  "gene_symbol": "CUX2"
}